hippocampal neuron apoptotic process [GO:0110088] (biological process) Relationships: is a type of neuron apoptotic process [GO:0051402] References: PMID:18940801 Sources: GOC:sl Regulation: regulated by regulation of hippocampal neuron apoptotic process [GO:0110089]; positively regulated by GO:0110090; negatively regulated by negative regulation of hippocampal neuron apoptotic process [GO:0110091] Definition: Any apoptotic process that occurs in a hippocampal neuron.